positive regulation of cardiac conduction [GO:1903781] (biological process) Definition: Any process that activates or increases the frequency, rate or extent of cardiac conduction. References: PMID:12967627 Sources: GOC:BHF, GOC:TermGenie, GOC:mtg_cardiac_conduct_nov11, GOC:rph, GO_REF:0000058 Also known as: up regulation of cardiac conduction, up-regulation of cardiac conduction, upregulation of cardiac conduction, activation of cardiac conduction Relationships: is a type of positive regulation of biological process [GO:0048518]; is a type of regulation of cardiac conduction [GO:1903779]; positively regulates cardiac conduction [GO:0061337]